{
  "gene_symbol": "TBC1D17",
  "term_id": "GO:0042147",
  "gene": "UniProtKB:Q9HA65",
  "term_label": "retrograde transport, endosome to Golgi",
  "gene_name": "TBC1 domain family member 17"
}